{
  "term_label": "positive regulation of DNA-templated transcription",
  "gene_name": "Erythroid differentiation-related factor 1",
  "term_id": "GO:0045893",
  "gene": "UniProtKB:Q3B7T1",
  "gene_symbol": "EDRF1"
}